{
  "term_id": "GO:0030127",
  "gene_symbol": "SEC13",
  "gene": "UniProtKB:P55735",
  "term_label": "COPII vesicle coat",
  "gene_name": "Protein SEC13 homolog"
}